{
  "term_id": "UNKNOWN:0001",
  "gene": "UniProtKB:Q8N0V3",
  "term_label": "Unknown molecular function",
  "gene_symbol": "RBFA",
  "gene_name": "Putative ribosome-binding factor A, mitochondrial"
}